{
  "term_label": "type I interferon-mediated signaling pathway",
  "gene_symbol": "OASL",
  "gene": "UniProtKB:Q15646",
  "gene_name": "2'-5'-oligoadenylate synthase-like protein",
  "term_id": "GO:0060337"
}